{
  "term_id": "GO:0089701",
  "gene": "UniProtKB:Q01081",
  "term_label": "U2AF complex",
  "gene_symbol": "U2AF1",
  "gene_name": "Splicing factor U2AF 35 kDa subunit"
}